{
  "gene_symbol": "GABBR2",
  "term_id": "GO:0007214",
  "term_label": "gamma-aminobutyric acid signaling pathway",
  "gene": "UniProtKB:O75899",
  "gene_name": "Gamma-aminobutyric acid type B receptor subunit 2"
}